{
  "gene_symbol": "TDRD9",
  "gene": "UniProtKB:Q8NDG6",
  "term_label": "cytoplasm",
  "gene_name": "ATP-dependent RNA helicase TDRD9",
  "term_id": "GO:0005737"
}